polymeric cytoskeletal fiber [GO:0099513] (cellular component) Definition: A component of the cytoskeleton consisting of a homo or heteropolymeric fiber constructed from an indeterminate number of protein subunits. Sources: GOC:dos Relationships: is_a GO:0099512; is part of cytoskeleton [GO:0005856] Subtypes: outer dense fiber [GO:0001520], GO:0005874, intermediate filament [GO:0005882], actin filament [GO:0005884]